{
  "gene_symbol": "EGFL7",
  "term_id": "GO:0001570",
  "gene_name": "Epidermal growth factor-like protein 7",
  "gene": "UniProtKB:Q9UHF1",
  "term_label": "vasculogenesis"
}